{
  "gene": "UniProtKB:P01584",
  "gene_name": "Interleukin-1 beta",
  "gene_symbol": "IL1B",
  "term_id": "GO:0006955",
  "term_label": "immune response"
}